{
  "term_id": "UNKNOWN:0002",
  "gene_symbol": "DPF3",
  "term_label": "Unknown biological process",
  "gene": "UniProtKB:Q92784",
  "gene_name": "Zinc finger protein DPF3"
}